{
  "gene_name": "Heat shock-related 70 kDa protein 2",
  "term_label": "protein refolding",
  "gene": "UniProtKB:P54652",
  "gene_symbol": "HSPA2",
  "term_id": "GO:0042026"
}